{
  "gene": "UniProtKB:A8MVZ5",
  "gene_symbol": "BTNL10P",
  "gene_name": "Putative butyrophilin-like protein 10 pseudogene",
  "term_label": "regulation of cytokine production",
  "term_id": "GO:0001817"
}